fluoride channel activity [GO:0062054] (molecular function) Relationships: is a type of monoatomic anion channel activity [GO:0005253]; is a type of GO:1903425 Definition: Enables the energy-independent facilitated diffusion of a fluoride ion through a transmembrane aqueous pore or channel. References: PMID:23991286, PMID:25156118